{
  "term_label": "plasma membrane",
  "gene": "UniProtKB:Q12879",
  "term_id": "GO:0005886",
  "gene_symbol": "GRIN2A",
  "gene_name": "Glutamate receptor ionotropic, NMDA 2A"
}